{
  "term_label": "phosphatidylethanolamine biosynthetic process",
  "gene_symbol": "ETNK2",
  "term_id": "GO:0006646",
  "gene": "UniProtKB:Q9NVF9",
  "gene_name": "Ethanolamine kinase 2"
}